regulation of presynaptic cytosolic calcium ion concentration [GO:0099509] (biological process) Sources: GOC:dos Also known as: regulation of presynaptic cytosolic calcium levels Definition: Any process that regulates the concentration of calcium in the presynaptic cytosol. Relationships: is a type of regulation of cytosolic calcium ion concentration [GO:0051480]; is a type of neuron cellular homeostasis [GO:0070050]; BFO_0000066 presynapse [GO:0098793]